{
  "gene_symbol": "IFNA6",
  "gene_name": "Interferon alpha-6",
  "term_id": "GO:0002286",
  "gene": "UniProtKB:P05013",
  "term_label": "T cell activation involved in immune response"
}